{
  "gene_name": "Peptidyl-prolyl cis-trans isomerase FKBP1A",
  "gene": "UniProtKB:P62942",
  "term_id": "GO:0006457",
  "gene_symbol": "FKBP1A",
  "term_label": "protein folding"
}